phloem unloading [GO:0110127] (biological process) Relationships: is a type of phloem transport [GO:0010233] Definition: The process of unloading solutes that are produced in the source tissues, from the sieve tube or companion cell of the phloem into the sink tissues. References: PMID:19025382 Sources: GOC:lr Subtypes: GO:0110128